aminophospholipid transport [GO:0015917] (biological process) Definition: The directed movement of aminophospholipids into, out of or within a cell, or between cells, by means of some agent such as a transporter or pore. Aminophospholipids contain phosphoric acid as a mono- or diester and an amino (NH2) group. Sources: GOC:ai Relationships: is a type of phospholipid transport [GO:0015914]; is a type of nitrogen compound transport [GO:0071705] Subtypes: aminophospholipid translocation [GO:0140331]